AP-3 adaptor complex binding [GO:0035651] (molecular function) References: PMID:21097499 Definition: Binding to an AP-3 adaptor complex. The AP-3 adaptor complex is a heterotetrameric AP-type membrane coat adaptor complex that consists of beta3, delta, mu3 and sigma3 subunits and is found associated with endosomal membranes. In at least humans, the AP-3 complex can be heterogeneric due to the existence of multiple subunit isoforms encoded by different genes (beta3A and beta3B, mu3A and mu3B, and sigma3A and sigma3B). Relationships: is a type of protein-containing complex binding [GO:0044877]